recombinational interstrand cross-link repair [GO:0036298] (biological process) References: PMID:20658649 Sources: GOC:vw Relationships: is a type of GO:0000725; is a type of interstrand cross-link repair [GO:0036297] Also known as: recombination-dependent interstrand cross-link repair, Fanconi pathway Definition: Removal of a DNA interstrand crosslink (a covalent attachment of DNA bases on opposite strands of the DNA) and restoration of the DNA by a mechanism that involves the exchange, reciprocal or nonreciprocal, of genetic material between the broken DNA molecule and a homologous DNA region.